{
  "term_label": "positive regulation of cholesterol storage",
  "gene_name": "Sterol regulatory element-binding protein 2",
  "term_id": "GO:0010886",
  "gene": "UniProtKB:Q12772",
  "gene_symbol": "SREBF2"
}